{
  "gene": "UniProtKB:Q14257",
  "term_label": "Unknown biological process",
  "gene_name": "Reticulocalbin-2",
  "term_id": "UNKNOWN:0002",
  "gene_symbol": "RCN2"
}